{
  "gene_symbol": "GIT1",
  "term_label": "synapse",
  "gene": "UniProtKB:Q9Y2X7",
  "term_id": "GO:0045202",
  "gene_name": "ARF GTPase-activating protein GIT1"
}